protein K69-linked ufmylation [GO:1990592] (biological process) Definition: A protein ufmylation process in which a polymer of the ubiquitin-like protein UFM1 is formed by linkages between lysine residues at position 69 of the UFM1 monomers, is added to a protein. Relationships: is a type of GO:1990564 References: PMID:25219498